{
  "gene_name": "E3 ubiquitin-protein ligase RNF4",
  "gene": "UniProtKB:P78317",
  "term_label": "positive regulation of transcription by RNA polymerase II",
  "gene_symbol": "RNF4",
  "term_id": "GO:0045944"
}